{
  "gene_symbol": "PLXNB2",
  "gene_name": "Plexin-B2",
  "term_id": "GO:0002116",
  "term_label": "semaphorin receptor complex",
  "gene": "UniProtKB:O15031"
}